{
  "gene_name": "Histone acetyltransferase KAT2B",
  "gene_symbol": "KAT2B",
  "term_label": "histone H3 acetyltransferase activity",
  "gene": "UniProtKB:Q92831",
  "term_id": "GO:0010484"
}